{
  "gene_symbol": "CASC3",
  "term_id": "UNKNOWN:0001",
  "gene": "UniProtKB:O15234",
  "gene_name": "Protein CASC3",
  "term_label": "Unknown molecular function"
}